{
  "term_id": "GO:0005102",
  "gene": "UniProtKB:O75636",
  "gene_symbol": "FCN3",
  "gene_name": "Ficolin-3",
  "term_label": "signaling receptor binding"
}